regulation of pancreatic stellate cell proliferation [GO:2000229] (biological process) Sources: GOC:mah Relationships: is a type of regulation of fibroblast proliferation [GO:0048145]; regulates GO:0072343 Subtypes: GO:2000230, positive regulation of pancreatic stellate cell proliferation [GO:2000231] Definition: Any process that modulates the frequency, rate or extent of pancreatic stellate cell proliferation.